{
  "gene_symbol": "BRD3",
  "term_label": "histone binding",
  "gene_name": "Bromodomain-containing protein 3",
  "term_id": "GO:0042393",
  "gene": "UniProtKB:Q15059"
}